creatine kinase activity [GO:0004111] (molecular function) Also known as: ATP:creatine N-phosphotransferase activity, ATP:creatine phosphotransferase activity, BB-CK, CK, CK-BB, CK-MB, CK-MM, CKMiMi, MB-CK, MM-CK, Mi-CK, MiMi-CK, adenosine triphosphate-creatine transphosphorylase activity, creatine phosphokinase activity, creatine phosphotransferase activity, phosphocreatine kinase activity Definition: Catalysis of the reaction: ATP + creatine = N-phosphocreatine + ADP + 2 H+. Sources: EC:2.7.3.2, RHEA:17157 Note: Note that this term has a MetaCyc pathway reference as the pathway only has a single step. Relationships: is a type of GO:0016301; is a type of phosphotransferase activity, nitrogenous group as acceptor [GO:0016775]